{
  "term_id": "GO:0030154",
  "gene_symbol": "NR2F6",
  "gene_name": "Nuclear receptor subfamily 2 group F member 6",
  "gene": "UniProtKB:P10588",
  "term_label": "cell differentiation"
}